AP-1 adaptor complex binding [GO:0035650] (molecular function) References: PMID:21097499 Relationships: is a type of protein-containing complex binding [GO:0044877] Definition: Binding to an AP-1 adaptor complex. The AP-1 adaptor complex is a heterotetrameric AP-type membrane coat adaptor complex that consists of beta1, gamma, mu1 and sigma1 subunits and links clathrin to the membrane surface of a vesicle. In at least humans, the AP-1 complex can be heterogeneric due to the existence of multiple subunit isoforms encoded by different genes (gamma1 and gamma2, mu1A and mu1B, and sigma1A, sigma1B and sigma1C).